{
  "gene_symbol": "EFL1",
  "term_label": "GTPase activity",
  "gene": "UniProtKB:Q7Z2Z2",
  "gene_name": "Elongation factor-like GTPase 1",
  "term_id": "GO:0003924"
}